{
  "gene": "UniProtKB:Q8N9F8",
  "term_label": "DNA-binding transcription factor activity, RNA polymerase II-specific",
  "term_id": "GO:0000981",
  "gene_symbol": "ZNF454",
  "gene_name": "Zinc finger protein 454"
}